germacrene-A synthase activity [GO:0034005] (molecular function) Also known as: (+)-(10R)-germacrene A synthase activity, (+)-germacrene A synthase activity, 2-trans,6-trans-farnesyl-diphosphate diphosphate-lyase (germacrene-A-forming) activity, 2-trans,6-trans-farnesyl-diphosphate diphosphate-lyase [(+)-germacrene-A-forming] activity, GAS, germacrene A synthase activity Relationships: is a type of sesquiterpene synthase activity [GO:0010334] Sources: EC:4.2.3.23, RHEA:12516 Definition: Catalysis of the reaction: 2-trans,6-trans-farnesyl diphosphate = (+)-(R)-germacrene A + diphosphate.